regulation of mast cell degranulation [GO:0043304] (BP) Subtypes: negative regulation of mast cell degranulation [GO:0043305], positive regulation of mast cell degranulation [GO:0043306] Relationships: is a type of regulation of myeloid leukocyte mediated immunity [GO:0002886]; is a type of regulation of leukocyte degranulation [GO:0043300]; regulates mast cell degranulation [GO:0043303] Also known as: regulation of mast cell granule exocytosis Sources: ISBN:0781735149 Definition: Any process that modulates the frequency, rate, or extent of mast cell degranulation.